{
  "term_label": "positive regulation of non-canonical NF-kappaB signal transduction",
  "gene_symbol": "TRIP6",
  "gene": "UniProtKB:Q15654",
  "term_id": "GO:1901224",
  "gene_name": "Thyroid receptor-interacting protein 6"
}